2-oxo-3-(5-oxofuran-2-ylidene)propanoate lactonase activity [GO:0102355] (molecular function) Sources: EC:3.1.1.91, GOC:pz Relationships: is a type of GO:0052689 Definition: Catalysis of the reaction: 2-oxo-3-(5-oxofuran-2-ylidene)propanoate + H2O = 3-maleylpyruvate + H+.